{
  "term_id": "GO:0007605",
  "term_label": "sensory perception of sound",
  "gene": "UniProtKB:Q7Z7J7",
  "gene_symbol": "LHFPL4",
  "gene_name": "LHFPL tetraspan subfamily member 4 protein"
}